{
  "term_label": "cytoplasm",
  "gene_symbol": "ARHGAP19",
  "gene": "UniProtKB:Q14CB8",
  "term_id": "GO:0005737",
  "gene_name": "Rho GTPase-activating protein 19"
}